{
  "term_id": "GO:0006355",
  "gene_symbol": "HMGA2",
  "term_label": "regulation of DNA-templated transcription",
  "gene_name": "High mobility group protein HMGI-C",
  "gene": "UniProtKB:P52926"
}